{
  "term_label": "plasma membrane",
  "term_id": "GO:0005886",
  "gene_symbol": "ARVCF",
  "gene": "UniProtKB:O00192",
  "gene_name": "Splicing regulator ARVCF"
}